{
  "gene": "UniProtKB:Q96AQ2",
  "gene_name": "Transmembrane protein 125",
  "term_id": "UNKNOWN:0001",
  "gene_symbol": "TMEM125",
  "term_label": "Unknown molecular function"
}